{
  "gene": "UniProtKB:Q96GA7",
  "term_label": "Unknown cellular component",
  "gene_symbol": "SDSL",
  "gene_name": "Serine dehydratase-like",
  "term_id": "UNKNOWN:0003"
}